dehydroaustinol biosynthetic process [GO:1900563] (biological process) Also known as: dehydroaustinol anabolism, dehydroaustinol biosynthesis, dehydroaustinol formation, dehydroaustinol synthesis Regulation: regulated by GO:1900649; negatively regulated by negative regulation of dehydroaustinol biosynthetic process [GO:1900650]; positively regulated by positive regulation of dehydroaustinol biosynthetic process [GO:1900651] Relationships: is a type of secondary metabolite biosynthetic process [GO:0044550] Sources: GOC:TermGenie, GOC:di Definition: The chemical reactions and pathways resulting in the formation of dehydroaustinol.